4,6-pyruvylated galactose residue biosynthetic process [GO:0051072] (biological process) Also known as: 4,6-pyruvylated galactose residue anabolism, 4,6-pyruvylated galactose residue biosynthesis, 4,6-pyruvylated galactose residue formation, 4,6-pyruvylated galactose residue synthesis, 4-6-O-[(R)(1-carboxyethylidine)]-Gal-beta-1,3 biosynthesis, 4-6-O-[(R)(1-carboxyethylidine)]-Gal-beta-1,3 biosynthetic process, PvGal biosynthesis, PvGal biosynthetic process Regulation: regulated by regulation of 4,6-pyruvylated galactose residue biosynthetic process [GO:0060634] Definition: The chemical reactions and pathways resulting in the formation of the pyruvylated galactose residue 4-6-O-[(R)(1-carboxyethylidine)]-Gal-beta-1,3-. The galactose residue is part of a larger polysaccharide chain. Relationships: is a type of GO:0000271 References: PMID:15173185 Sources: GOC:ai